{
  "gene": "UniProtKB:Q5SZD4",
  "gene_name": "Glycine N-acyltransferase-like protein 3",
  "term_label": "glycine N-acyltransferase activity",
  "gene_symbol": "GLYATL3",
  "term_id": "GO:0047961"
}